{
  "gene": "UniProtKB:P59551",
  "term_label": "membrane",
  "gene_name": "Taste receptor type 2 member 60",
  "gene_symbol": "TAS2R60",
  "term_id": "GO:0016020"
}